regulation of arginine biosynthetic process via ornithine [GO:2000013] (biological process) Definition: Any process that modulates the frequency, rate or extent of arginine biosynthetic process via ornithine. Also known as: regulation of arginine anabolism via ornithine, regulation of arginine formation via ornithine, regulation of arginine synthesis via ornithine Sources: GOC:obol Relationships: is a type of regulation of arginine biosynthetic process [GO:1900079]; regulates L-arginine biosynthetic process via ornithine [GO:0042450]